{
  "gene": "UniProtKB:Q9Y272",
  "gene_symbol": "RASD1",
  "term_id": "GO:0031681",
  "gene_name": "Dexamethasone-induced Ras-related protein 1",
  "term_label": "G-protein beta-subunit binding"
}